{
  "gene_name": "Myelin protein zero-like protein 3",
  "gene_symbol": "MPZL3",
  "term_id": "GO:0005886",
  "gene": "UniProtKB:Q6UWV2",
  "term_label": "plasma membrane"
}